{
  "gene_symbol": "SYTL1",
  "term_id": "GO:0070382",
  "gene_name": "Synaptotagmin-like protein 1",
  "gene": "UniProtKB:Q8IYJ3",
  "term_label": "exocytic vesicle"
}